1,4-alpha-glucan branching enzyme activity [GO:0003844] (molecular function) Relationships: is_a hexosyltransferase activity [GO:0016758] Definition: Catalysis of the transfer of a segment of a (1->4)-alpha-D-glucan chain to a primary hydroxyl group in a similar glucan chain. Also known as: 1,4-alpha-D-glucan:1,4-alpha-D-glucan 6-alpha-D-(1,4-alpha-D-glucano)-transferase activity, 1,4-glucan-6-(1,4-glucano)-transferase activity, Q-enzyme, alpha-1,4-glucan:alpha-1,4-glucan-6-glycosyltransferase activity, alpha-glucan-branching glycosyltransferase activity, amylo-(1,4 to 1,6)transglucosidase activity, amylo-(1,4->1,6)-transglycosylase activity, amylose isomerase activity, branching enzyme activity, branching glycosyltransferase activity, enzymatic branching factor, enzyme Q, glucosan transglycosylase activity, glycogen branching enzyme activity, plant branching enzyme, starch branching enzyme Sources: EC:2.4.1.18